protein targeting to membrane [GO:0006612] (BP) Regulation: regulated by regulation of protein targeting to membrane [GO:0090313]; positively regulated by GO:0090314; negatively regulated by negative regulation of protein targeting to membrane [GO:0090315] Subtypes: cotranslational protein targeting to membrane [GO:0006613], post-translational protein targeting to endoplasmic reticulum membrane [GO:0006620], protein targeting to vacuolar membrane [GO:0044395] Relationships: is a type of protein targeting [GO:0006605]; is a type of GO:0090150 Definition: The process of directing proteins towards a membrane, usually using signals contained within the protein. Sources: GOC:curators Also known as: protein membrane targeting, protein-membrane targeting